SAM domain binding [GO:0032093] (MF) Definition: Binding to a SAM (Sterile Alpha Motif) domain, which is a 70-amino acid protein sequence that participates in protein-protein, protein-lipid, and protein-RNA interactions and is conserved from lower to higher eukaryotes. References: PMID:16337230 Sources: GOC:mcc Also known as: Sterile Alpha Motif domain binding Relationships: is a type of protein domain specific binding [GO:0019904]